{
  "term_label": "nucleus",
  "gene_name": "Tumor protein p53-inducible nuclear protein 1",
  "gene_symbol": "TP53INP1",
  "term_id": "GO:0005634",
  "gene": "UniProtKB:Q96A56"
}